{
  "gene_name": "Programmed cell death protein 5",
  "term_label": "Unknown molecular function",
  "gene_symbol": "PDCD5",
  "term_id": "UNKNOWN:0001",
  "gene": "UniProtKB:O14737"
}